{
  "gene": "UniProtKB:Q9NPC6",
  "term_label": "telethonin binding",
  "gene_name": "Myozenin-2",
  "gene_symbol": "MYOZ2",
  "term_id": "GO:0031433"
}